{
  "term_id": "GO:0030832",
  "gene_name": "Myosin-IIIa",
  "term_label": "regulation of actin filament length",
  "gene_symbol": "MYO3A",
  "gene": "UniProtKB:Q8NEV4"
}